{
  "gene": "UniProtKB:O96005",
  "gene_name": "Putative lipid scramblase CLPTM1",
  "gene_symbol": "CLPTM1",
  "term_id": "GO:0012505",
  "term_label": "endomembrane system"
}